{
  "term_id": "GO:0003682",
  "term_label": "chromatin binding",
  "gene_name": "Metal-response element-binding transcription factor 2",
  "gene_symbol": "MTF2",
  "gene": "UniProtKB:Q9Y483"
}